{
  "term_id": "GO:0005737",
  "term_label": "cytoplasm",
  "gene_name": "G2_mitotic-specific cyclin-B3",
  "gene_symbol": "CCNB3",
  "gene": "UniProtKB:Q8WWL7"
}